{
  "term_label": "protein folding",
  "gene": "UniProtKB:A0A075B767",
  "gene_symbol": "PPIAL4H",
  "term_id": "GO:0006457",
  "gene_name": "Peptidyl-prolyl cis-trans isomerase A-like 4H"
}